{
  "gene_symbol": "RUNX2",
  "gene": "UniProtKB:Q13950",
  "term_label": "DNA-binding transcription factor activity, RNA polymerase II-specific",
  "gene_name": "Runt-related transcription factor 2",
  "term_id": "GO:0000981"
}